{
  "gene_symbol": "PEX1",
  "term_label": "ATP hydrolysis activity",
  "gene": "UniProtKB:O43933",
  "gene_name": "Peroxisomal ATPase PEX1",
  "term_id": "GO:0016887"
}